alpha,alpha-trehalose-phosphate synthase complex (UDP-forming) [GO:0005946] (cellular component) Definition: A protein complex that possesses alpha,alpha-trehalose-phosphate synthase (UDP-forming) and trehalose-phosphatase activities, and thus catalyzes two reactions in trehalose biosynthesis. In the complex identified in Saccharomyces, Tps1p has alpha,alpha-trehalose-phosphate synthase (UDP-forming) activity, Tps2p has trehalose 6-phosphate phosphatase activity; Tps3p is a regulatory subunit, and an additional subunit, Tsl1p, may be present. Note: See also the molecular function term 'alpha,alpha-trehalose-phosphate synthase (UDP-forming) activity ; GO:0003825'. Also known as: UDP-glucose-glucosephosphate glucosyltransferase complex, trehalose-6-phosphate synthase complex, trehalose-6-phosphate synthase/phosphatase Relationships: is a type of transferase complex [GO:1990234]; is part of cytoplasm [GO:0005737] References: PMID:9837904